{
  "term_id": "UNKNOWN:0002",
  "gene_name": "Probable non-functional T cell receptor gamma variable 10",
  "gene": "UniProtKB:A0A0A0MS01",
  "gene_symbol": "TRGV10",
  "term_label": "Unknown biological process"
}